{
  "gene_name": "Putative taste receptor type 2 member 36",
  "gene_symbol": "TAS2R36",
  "term_label": "Unknown molecular function",
  "term_id": "UNKNOWN:0001",
  "gene": "UniProtKB:P0DTE0"
}